{
  "gene_symbol": "NR2C1",
  "gene_name": "Nuclear receptor subfamily 2 group C member 1",
  "term_label": "nuclear receptor activity",
  "term_id": "GO:0004879",
  "gene": "UniProtKB:P13056"
}